U3 snoRNA binding [GO:0034511] (molecular function) Definition: Binding to a U3 small nucleolar RNA. Sources: GOC:mah Relationships: is a type of snoRNA binding [GO:0030515]